{
  "gene": "UniProtKB:Q86VD1",
  "term_id": "UNKNOWN:0001",
  "gene_name": "MORC family CW-type zinc finger protein 1",
  "term_label": "Unknown molecular function",
  "gene_symbol": "MORC1"
}